{
  "gene_symbol": "OR2T4",
  "gene": "UniProtKB:Q8NH00",
  "gene_name": "Olfactory receptor 2T4",
  "term_id": "GO:0050911",
  "term_label": "detection of chemical stimulus involved in sensory perception of smell"
}